regulation of systemic arterial blood pressure by carotid body chemoreceptor signaling [GO:0003027] (biological process) Definition: The process that modulates blood pressure by the action of chemoreceptors found in the carotid bodies and their resultant modulation of the vasomotor center. Chemoreceptors respond to oxygen, carbon dioxide and hydrogen ions. Relationships: is a type of GO:0001979 Also known as: vagal reflex, carotid body chemoreceptor regulation of systemic arterial blood pressure, carotid body chemoreceptor response to lowering of systemic arterial blood pressure, regulation of systemic arterial blood pressure by carotid body chemoreceptor signalling Sources: GOC:dph, GOC:mtg_cardio, GOC:tb